nuclease activator activity [GO:0170053] (molecular function) References: PMID:24736845 Subtypes: endodeoxyribonuclease activator activity [GO:0140656], GO:0170054 Relationships: is a type of enzyme activator activity [GO:0008047]; positively regulates nuclease activity [GO:0004518] Definition: Binds to and increases the activity of a nuclease.